{
  "gene": "UniProtKB:A0A8Q3WKH5",
  "term_label": "nucleus",
  "gene_symbol": "H2AL1Q",
  "term_id": "GO:0005634",
  "gene_name": "Histone H2A"
}